{
  "gene_name": "CCR4-NOT transcription complex subunit 3",
  "gene": "UniProtKB:O75175",
  "gene_symbol": "CNOT3",
  "term_label": "P-body",
  "term_id": "GO:0000932"
}